negative regulation of calcium ion import [GO:0090281] (biological process) Relationships: is a type of negative regulation of calcium ion transport [GO:0051926]; is a type of GO:0090279; negatively regulates calcium ion import [GO:0070509] Also known as: negative regulation of transmembrane calcium influx Definition: Any process that decreases the rate, frequency, or extent of the directed movement of calcium ions into a cell or organelle. Sources: GOC:BHF Subtypes: negative regulation of calcium ion import across plasma membrane [GO:1905949]